{
  "gene_symbol": "ICAM5",
  "term_label": "plasma membrane",
  "gene": "UniProtKB:Q9UMF0",
  "term_id": "GO:0005886",
  "gene_name": "Intercellular adhesion molecule 5"
}